{
  "gene_symbol": "TIGAR",
  "gene": "UniProtKB:Q9NQ88",
  "gene_name": "Fructose-2,6-bisphosphatase TIGAR",
  "term_label": "negative regulation of glycolytic process",
  "term_id": "GO:0045820"
}